{
  "gene": "UniProtKB:Q9Y2G8",
  "gene_symbol": "DNAJC16",
  "term_id": "UNKNOWN:0002",
  "term_label": "Unknown biological process",
  "gene_name": "DnaJ homolog subfamily C member 16"
}